{
  "gene_symbol": "MFI",
  "term_id": "UNKNOWN:0003",
  "gene_name": "Protein MFI",
  "gene": "UniProtKB:Q8NCR3",
  "term_label": "Unknown cellular component"
}